{
  "term_label": "regulation of organelle assembly",
  "gene_symbol": "EZR",
  "gene_name": "Ezrin",
  "term_id": "GO:1902115",
  "gene": "UniProtKB:P15311"
}